{
  "gene_name": "Diacylglycerol lipase-beta",
  "gene": "UniProtKB:Q8NCG7",
  "term_label": "arachidonate metabolic process",
  "term_id": "GO:0019369",
  "gene_symbol": "DAGLB"
}